{
  "gene_name": "Forkhead box protein R1",
  "gene_symbol": "FOXR1",
  "term_label": "Unknown biological process",
  "term_id": "UNKNOWN:0002",
  "gene": "UniProtKB:Q6PIV2"
}